protein localization to outer membrane [GO:0089705] (biological process) Relationships: is a type of protein localization to membrane [GO:0072657]; is a type of protein localization to cell periphery [GO:1990778] Definition: A process in which a protein is transported to, or maintained in, a specific location the cell outer membrane. References: PMID:12823819 Sources: GOC:dos